proton motive force-driven motor activity [GO:0140605] (molecular function) References: PMID:18216858 Relationships: is a type of cytoskeletal motor activity [GO:0003774] Definition: A motor activity driven by an electrochemical proton gradient (proton-motive force). PMF-driven motors are used by bacterial flagella.